chromatin remodeling [GO:0006338] (biological process) Relationships: is a type of chromatin organization [GO:0006325] Also known as: chromatin modeling, chromatin modelling, chromatin remodelling, ATP-dependent chromatin remodeling, ATP-dependent chromatin remodelling References: PMID:12042764, PMID:12697820 Sources: GOC:jid, GOC:vw Subtypes: nucleosome organization [GO:0034728], epigenetic regulation of gene expression [GO:0040029], R-loop processing [GO:0062176], GO:0140673, GO:0140861, CENP-A eviction from euchromatin [GO:0140898] Definition: A dynamic process of chromatin reorganization resulting in changes to chromatin structure. These changes allow DNA metabolic processes such as transcriptional regulation, DNA recombination, DNA repair, and DNA replication.